{
  "term_label": "Unknown molecular function",
  "gene": "UniProtKB:O76080",
  "term_id": "UNKNOWN:0001",
  "gene_symbol": "ZFAND5",
  "gene_name": "AN1-type zinc finger protein 5"
}